{
  "gene": "UniProtKB:Q499Y3",
  "term_label": "Unknown molecular function",
  "gene_symbol": "Q499Y3",
  "term_id": "UNKNOWN:0001",
  "gene_name": "Putative uncharacterized protein C10orf88-like"
}